response to cesium ion [GO:0010164] (biological process) Subtypes: cellular response to cesium ion [GO:0071278] Definition: Any process that results in a change in state or activity of a cell or an organism (in terms of movement, secretion, enzyme production, gene expression, etc.) as a result of a cesium stimulus. Also known as: response to cesium Sources: GOC:sm Relationships: is a type of GO:0010038